{
  "gene_symbol": "SYK",
  "gene": "UniProtKB:P43405",
  "term_label": "positive regulation of cell adhesion mediated by integrin",
  "term_id": "GO:0033630",
  "gene_name": "Tyrosine-protein kinase SYK"
}